{
  "term_id": "GO:0043161",
  "gene": "UniProtKB:Q9UK73",
  "gene_symbol": "FEM1B",
  "term_label": "proteasome-mediated ubiquitin-dependent protein catabolic process",
  "gene_name": "Protein fem-1 homolog B"
}